{
  "gene": "UniProtKB:Q9H2B2",
  "term_id": "GO:0006906",
  "gene_symbol": "SYT4",
  "term_label": "vesicle fusion",
  "gene_name": "Synaptotagmin-4"
}